creatinase activity [GO:0016980] (molecular function) Relationships: is a type of hydrolase activity, acting on carbon-nitrogen (but not peptide) bonds, in linear amidines [GO:0016813] Also known as: creatine amidinohydrolase activity Definition: Catalysis of the reaction: creatine + H2O = sarcosine + urea. Sources: EC:3.5.3.3, RHEA:22456